glutamine biosynthetic process [GO:0006542] (biological process) Relationships: is a type of GO:0006541; is a type of glutamine family amino acid biosynthetic process [GO:0009084] Definition: The chemical reactions and pathways resulting in the formation of glutamine, 2-amino-4-carbamoylbutanoic acid. Also known as: glutamine anabolism, glutamine biosynthesis, glutamine formation, glutamine synthesis Sources: GOC:ai Subtypes: L-glutamine biosynthetic process [GO:1901704]